{
  "gene_symbol": "IER2",
  "term_label": "Unknown cellular component",
  "term_id": "UNKNOWN:0003",
  "gene": "UniProtKB:Q9BTL4",
  "gene_name": "Immediate early response gene 2 protein"
}